{
  "gene_name": "Putative uncharacterized protein FLJ45840",
  "term_id": "UNKNOWN:0002",
  "gene_symbol": "Q6ZS46",
  "gene": "UniProtKB:Q6ZS46",
  "term_label": "Unknown biological process"
}